{
  "gene_symbol": "PRRC1",
  "term_id": "GO:0005737",
  "gene": "UniProtKB:Q96M27",
  "gene_name": "Protein PRRC1",
  "term_label": "cytoplasm"
}